{
  "gene": "UniProtKB:Q8WUT4",
  "term_label": "Unknown molecular function",
  "gene_symbol": "LRRN4",
  "gene_name": "Leucine-rich repeat neuronal protein 4",
  "term_id": "UNKNOWN:0001"
}